{
  "gene": "UniProtKB:Q96AQ9",
  "term_id": "UNKNOWN:0003",
  "gene_name": "Protein FAM131C",
  "gene_symbol": "FAM131C",
  "term_label": "Unknown cellular component"
}